{
  "gene": "UniProtKB:Q5T3U5",
  "term_id": "GO:0008559",
  "gene_symbol": "ABCC10",
  "gene_name": "ATP-binding cassette sub-family C member 10",
  "term_label": "ABC-type xenobiotic transporter activity"
}